positive regulation of viral translation [GO:1904973] (biological process) Definition: Any process that activates or increases the frequency, rate or extent of viral translation. References: PMID:19666601 Sources: GOC:TermGenie, GOC:bhm, GO_REF:0000058 Also known as: positive regulation of viral protein anabolism, positive regulation of viral protein biosynthesis, positive regulation of viral protein biosynthetic process, positive regulation of viral protein formation, positive regulation of viral protein synthesis, up regulation of viral protein anabolism, up regulation of viral protein biosynthesis, up regulation of viral protein biosynthetic process, up regulation of viral protein formation, up regulation of viral protein synthesis, up regulation of viral translation, up-regulation of viral protein anabolism, up-regulation of viral protein biosynthesis, up-regulation of viral protein biosynthetic process, up-regulation of viral protein formation, up-regulation of viral protein synthesis, up-regulation of viral translation, upregulation of viral protein anabolism, upregulation of viral protein biosynthesis, upregulation of viral protein biosynthetic process, upregulation of viral protein formation, upregulation of viral protein synthesis, upregulation of viral translation, activation of viral protein anabolism, activation of viral protein biosynthesis, activation of viral protein biosynthetic process, activation of viral protein formation, activation of viral protein synthesis, activation of viral translation Relationships: is a type of positive regulation of viral process [GO:0048524]; is_a regulation of viral translation [GO:1904971]; RO_0002213 viral translation [GO:0019081]